{
  "term_id": "GO:0036402",
  "gene": "UniProtKB:P62191",
  "gene_name": "26S proteasome regulatory subunit 4",
  "gene_symbol": "PSMC1",
  "term_label": "proteasome-activating activity"
}